S-adenosyl-L-methionine transport [GO:0015805] (biological process) Sources: GOC:ai Relationships: is a type of organic cation transport [GO:0015695]; is a type of sulfur compound transport [GO:0072348] Definition: The directed movement of S-adenosylmethionine, S-(5'-adenosyl)-L-methionine, an important intermediate in one-carbon metabolism, into, out of or within a cell, or between cells, by means of some agent such as a transporter or pore. Subtypes: S-adenosyl-L-methionine transmembrane transport [GO:1901962] Also known as: S-adenosyl methionine transport, S-adenosylmethionine transport, SAM transport